{
  "term_id": "UNKNOWN:0002",
  "gene_symbol": "YWHAH-AS1",
  "gene_name": "Putative uncharacterized protein YWHAH-AS1",
  "gene": "UniProtKB:Q9Y442",
  "term_label": "Unknown biological process"
}